{
  "gene": "UniProtKB:Q07065",
  "gene_name": "Cytoskeleton-associated protein 4",
  "term_id": "UNKNOWN:0002",
  "term_label": "Unknown biological process",
  "gene_symbol": "CKAP4"
}